histone binding [GO:0042393] (molecular function) Relationships: is a type of protein binding [GO:0005515] References: PMID:16209651, PMID:30212449, PMID:9305837 Sources: GOC:jl Definition: Binding to a histone, any of a group of water-soluble proteins found in association with the DNA of eukaryotic or archaeal chromosomes. They are involved in the condensation and coiling of chromosomes during cell division and have also been implicated in gene regulation and DNA replication. They may be chemically modified (methylated, acetlyated and others) to regulate gene transcription. Also known as: histone-specific chaperone activity